{
  "gene_name": "Putative uncharacterized protein TSPEAR-AS2",
  "gene": "UniProtKB:P59090",
  "term_label": "Unknown biological process",
  "gene_symbol": "TSPEAR-AS2",
  "term_id": "UNKNOWN:0002"
}